regulation of transepithelial transport [GO:0150111] (biological process) References: PMID:27593915 Sources: GOC:aruk Relationships: is a type of GO:0051049; RO_0002211 transepithelial transport [GO:0070633] Definition: Any process that modulates the frequency, rate or extent of transepithelial transport.